hydrocarbon metabolic process [GO:0120252] (biological process) Definition: The chemical reactions and pathways involving a hydrocarbon, a compound consisting of carbon and hydrogen only. Sources: GOC:krc, Wikipedia:Hydrocarbon Also known as: hydrocarbon metabolism Relationships: is_a metabolic process [GO:0008152] Subtypes: methane metabolic process [GO:0015947], GO:0018910, GO:0018966, GO:0018970, terpene metabolic process [GO:0042214], hydrocarbon biosynthetic process [GO:0120251], hydrocarbon catabolic process [GO:0120253], tridecane metabolic process [GO:1900631], GO:1900633, heptadecane metabolic process [GO:1900635], olefin metabolic process [GO:1900673]